cell migration in hindbrain [GO:0021535] (biological process) Sources: GOC:cls, GOC:dgh, GOC:dph, GOC:jid, GO_REF:0000021 Definition: The orderly movement of a cell that will reside in the hindbrain. Subtypes: hindbrain radial glia guided cell migration [GO:0021932], GO:0021934, deep nuclear neuron cell migration [GO:0021946], outward migration of deep nuclear neurons [GO:0021947], inward migration of deep nuclear neurons [GO:0021948], rhombomere cell migration [GO:0022035], GO:0035765 Relationships: is a type of cell migration [GO:0016477]; is part of hindbrain development [GO:0030902]